{
  "term_id": "GO:0019814",
  "gene_name": "Immunoglobulin lambda variable 4-3",
  "gene": "UniProtKB:A0A075B6K6",
  "gene_symbol": "IGLV4-3",
  "term_label": "immunoglobulin complex"
}